{
  "gene_symbol": "USP17L19",
  "gene": "UniProtKB:D6RCP7",
  "gene_name": "Ubiquitin carboxyl-terminal hydrolase 17-like protein 19",
  "term_id": "GO:0031647",
  "term_label": "regulation of protein stability"
}